cell activation involved in immune response [GO:0002263] (biological process) Definition: A change in the morphology or behavior of a cell resulting from exposure to an activating factor such as a cellular or soluble ligand, leading to the initiation or perpetuation of an immune response. Sources: GOC:add, GO_REF:0000022, ISBN:0781735149 Also known as: cell activation during immune response Relationships: is a type of cell activation [GO:0001775]; is a type of immune effector process [GO:0002252]; BFO_0000050 immune response [GO:0006955] Subtypes: endothelial cell activation involved in immune response [GO:0002264], astrocyte activation involved in immune response [GO:0002265], follicular dendritic cell activation involved in immune response [GO:0002267], leukocyte activation involved in immune response [GO:0002366]